{
  "gene_name": "Laminin subunit alpha-4",
  "gene": "UniProtKB:Q16363",
  "term_id": "GO:0005886",
  "gene_symbol": "LAMA4",
  "term_label": "plasma membrane"
}